{
  "gene_symbol": "COLEC12",
  "gene_name": "Collectin-12",
  "term_id": "GO:0038187",
  "term_label": "pattern recognition receptor activity",
  "gene": "UniProtKB:Q5KU26"
}